{
  "gene_symbol": "PRPH2",
  "term_id": "GO:0072659",
  "gene_name": "Peripherin-2",
  "term_label": "protein localization to plasma membrane",
  "gene": "UniProtKB:P23942"
}